{
  "term_id": "GO:0072534",
  "term_label": "perineuronal net",
  "gene_name": "Hyaluronan and proteoglycan link protein 4",
  "gene": "UniProtKB:Q86UW8",
  "gene_symbol": "HAPLN4"
}